{
  "gene_name": "PR domain-containing protein 11",
  "term_id": "GO:0005634",
  "gene_symbol": "PRDM11",
  "gene": "UniProtKB:Q9NQV5",
  "term_label": "nucleus"
}